{
  "gene_name": "Ubiquitin carboxyl-terminal hydrolase 13",
  "gene_symbol": "USP13",
  "term_id": "GO:0005634",
  "term_label": "nucleus",
  "gene": "UniProtKB:Q92995"
}